{
  "gene_name": "Cysteine dioxygenase type 1",
  "term_id": "GO:0008198",
  "gene_symbol": "CDO1",
  "gene": "UniProtKB:Q16878",
  "term_label": "ferrous iron binding"
}